negative regulation of intestinal epithelial cell development [GO:1905299] (biological process) Relationships: is a type of negative regulation of cell development [GO:0010721]; is a type of negative regulation of epithelial cell differentiation [GO:0030857]; is a type of GO:0051241; is_a GO:1905298; negatively regulates intestinal epithelial cell development [GO:0060576] Also known as: down regulation of intestinal epithelial cell development, down-regulation of intestinal epithelial cell development, downregulation of intestinal epithelial cell development, inhibition of intestinal epithelial cell development Definition: Any process that stops, prevents or reduces the frequency, rate or extent of intestinal epithelial cell development. References: PMID:23904268 Sources: GOC:BHF, GOC:BHF_miRNA, GOC:TermGenie, GOC:rph, GO_REF:0000058